{
  "gene_symbol": "NPIPB15",
  "term_label": "Unknown biological process",
  "term_id": "UNKNOWN:0002",
  "gene_name": "Nuclear pore complex-interacting protein family member B15",
  "gene": "UniProtKB:A6NHN6"
}